{
  "term_label": "proteolysis",
  "gene_symbol": "CAPN15",
  "term_id": "GO:0006508",
  "gene_name": "Calpain-15",
  "gene": "UniProtKB:O75808"
}